{
  "gene_symbol": "RAB17",
  "term_id": "GO:0006886",
  "term_label": "intracellular protein transport",
  "gene": "UniProtKB:Q9H0T7",
  "gene_name": "Ras-related protein Rab-17"
}